{
  "gene_symbol": "ZNF670",
  "term_id": "GO:0005634",
  "gene_name": "Zinc finger protein 670",
  "gene": "UniProtKB:Q9BS34",
  "term_label": "nucleus"
}